{
  "gene_name": "Coiled-coil domain-containing protein 179",
  "term_label": "Unknown biological process",
  "gene": "UniProtKB:H3BU77",
  "term_id": "UNKNOWN:0002",
  "gene_symbol": "CCDC179"
}